{
  "gene": "UniProtKB:Q9Y244",
  "term_id": "UNKNOWN:0001",
  "gene_name": "Proteasome maturation protein",
  "gene_symbol": "POMP",
  "term_label": "Unknown molecular function"
}